{
  "gene_symbol": "TNKS1BP1",
  "term_id": "GO:0000792",
  "term_label": "heterochromatin",
  "gene": "UniProtKB:Q9C0C2",
  "gene_name": "182 kDa tankyrase-1-binding protein"
}